{
  "gene_symbol": "C2CD5",
  "gene_name": "C2 domain-containing protein 5",
  "term_label": "intracellular protein transmembrane transport",
  "gene": "UniProtKB:Q86YS7",
  "term_id": "GO:0065002"
}